{
  "gene": "UniProtKB:Q9UKP3",
  "gene_symbol": "ITGB1BP2",
  "gene_name": "Integrin beta-1-binding protein 2",
  "term_id": "GO:0051298",
  "term_label": "centrosome duplication"
}